{
  "gene_symbol": "FRMD8P1",
  "gene": "UniProtKB:Q9BZ68",
  "term_label": "Unknown molecular function",
  "gene_name": "Putative FERM domain-containing protein FRMD8P1",
  "term_id": "UNKNOWN:0001"
}